{
  "term_label": "Unknown biological process",
  "gene": "UniProtKB:Q9H1Z4",
  "gene_symbol": "WDR13",
  "term_id": "UNKNOWN:0002",
  "gene_name": "WD repeat-containing protein 13"
}